regulation of circulating fibrinogen levels [GO:0044537] (biological process) Definition: Any process that modulates the quantity of fibrinogen circulating in the bloodstream. Sources: GOC:jl Subtypes: negative regulation of circulating fibrinogen levels [GO:0061754], GO:0061755 Relationships: is a type of regulation of biological quality [GO:0065008]